hydrolase activity, acting on carbon-nitrogen (but not peptide) bonds, in cyclic amides [GO:0016812] (molecular function) Relationships: is a type of hydrolase activity, acting on carbon-nitrogen (but not peptide) bonds [GO:0016810] Subtypes: allantoinase activity [GO:0004038], dihydroorotase activity [GO:0004151], dihydropyrimidinase activity [GO:0004157], beta-lactamase activity [GO:0008800], 5-oxoprolinase (ATP-hydrolyzing) activity [GO:0017168], epsilon-caprolactam lactamase activity [GO:0018752], cyanuric acid amidohydrolase activity [GO:0018753], GO:0019874, hydroxyisourate hydrolase activity [GO:0033971], enamidase activity [GO:0043792], imidazolone hydrolase activity [GO:0043804], xanthine hydrolase activity [GO:0043836], N-methylhydantoinase (ATP-hydrolyzing) activity [GO:0047423], 2,5-dioxopiperazine hydrolase activity [GO:0047532], barbiturase activity [GO:0047694], carboxymethylhydantoinase activity [GO:0047771], creatininase activity [GO:0047789], L-lysine-lactamase activity [GO:0050028], GO:0050480, GO:0050539 Sources: EC:3.5.2.- Definition: Catalysis of the hydrolysis of any non-peptide carbon-nitrogen bond in a cyclic amide.